organophosphate ester transport [GO:0015748] (biological process) Sources: GOC:mcc Definition: The directed movement of organophosphate esters into, out of or within a cell, or between cells, by means of some agent such as a transporter or pore. Organophosphate esters are small organic molecules containing phosphate ester bonds. Relationships: is a type of transport [GO:0006810] Subtypes: glycerophosphodiester transmembrane transport [GO:0001407], nucleotide transport [GO:0006862], hexose phosphate transport [GO:0015712], phosphoenolpyruvate transport [GO:0015714], GO:0015715, triose phosphate transport [GO:0015717], nucleotide-sugar transmembrane transport [GO:0015780], glycerol-3-phosphate transmembrane transport [GO:0015794], coenzyme A transport [GO:0015880], GO:0015914, GO:0015916, thiamine pyrophosphate transmembrane transport [GO:0030974], pyridoxal phosphate transport [GO:0031921], myo-inositol phosphate transport [GO:0033271], glycerol-2-phosphate transmembrane transport [GO:0070811]